{
  "gene_name": "Olfactory receptor 52B2",
  "gene": "UniProtKB:Q96RD2",
  "term_label": "olfactory receptor activity",
  "term_id": "GO:0004984",
  "gene_symbol": "OR52B2"
}